oligopeptide binding [GO:1900750] (molecular function) Subtypes: glutathione binding [GO:0043295], Ac-Asp-Glu binding [GO:1904492] Relationships: is a type of amide binding [GO:0033218] Definition: Binding to an oligopeptide. References: PMID:21854595 Sources: GOC:TermGenie Also known as: oligopeptides binding, Oligopeptid binding, oligopeptido binding